{
  "gene_symbol": "BCL11A",
  "term_label": "DNA-binding transcription factor activity",
  "gene": "UniProtKB:Q9H165",
  "gene_name": "B-cell lymphoma_leukemia 11A",
  "term_id": "GO:0003700"
}